{
  "term_label": "Unknown biological process",
  "gene_symbol": "CALHM3",
  "gene_name": "Calcium homeostasis modulator protein 3",
  "gene": "UniProtKB:Q86XJ0",
  "term_id": "UNKNOWN:0002"
}